3-deoxy-D-glycero-D-galacto-2-nonulosonic acid hydrolase activity [GO:0052791] (molecular function) Also known as: 2-keto-3-deoxynononic acid sialidase activity References: PMID:21247893 Sources: GOC:mengo_curators Relationships: is a type of alpha-sialidase activity [GO:0016997] Definition: Catalysis of the reaction: (2-keto-3-deoxynononic acid)n + H2O = (2-keto-3-deoxynononic acid)n-1 + 2-keto-3-deoxynononic acid. This reaction is the hydrolysis of a 2-keto-3-deoxynononic acid residue from a poly-2-keto-3-deoxynononic acid chain.